{
  "term_label": "chromatin",
  "gene_symbol": "CHD8",
  "gene": "UniProtKB:Q9HCK8",
  "gene_name": "Chromodomain-helicase-DNA-binding protein 8",
  "term_id": "GO:0000785"
}